{
  "term_id": "GO:0030687",
  "gene": "UniProtKB:Q6RFH5",
  "gene_symbol": "WDR74",
  "gene_name": "WD repeat-containing protein 74",
  "term_label": "preribosome, large subunit precursor"
}